{
  "gene": "UniProtKB:P32881",
  "term_label": "humoral immune response",
  "term_id": "GO:0006959",
  "gene_name": "Interferon alpha-8",
  "gene_symbol": "IFNA8"
}